mitochondrial outer membrane [GO:0005741] (cellular component) Also known as: mitochondrion outer membrane, outer mitochondrial membrane, outer mitochondrion membrane Definition: The outer, i.e. cytoplasm-facing, lipid bilayer of the mitochondrial envelope. Sources: GOC:ai Relationships: is a type of mitochondrial membrane [GO:0031966]; is a type of organelle outer membrane [GO:0031968]